{
  "term_label": "substrate adhesion-dependent cell spreading",
  "gene": "UniProtKB:Q9HBI1",
  "gene_symbol": "PARVB",
  "gene_name": "Beta-parvin",
  "term_id": "GO:0034446"
}